{
  "gene_symbol": "PRRT2",
  "term_id": "GO:0005886",
  "gene": "UniProtKB:Q7Z6L0",
  "term_label": "plasma membrane",
  "gene_name": "Proline-rich transmembrane protein 2"
}